{
  "gene": "UniProtKB:P29466",
  "gene_symbol": "CASP1",
  "gene_name": "Caspase-1",
  "term_id": "GO:0072559",
  "term_label": "NLRP3 inflammasome complex"
}